iodide peroxidase activity [GO:0004447] (molecular function) Also known as: TPO activity, iodinase activity, thyroid peroxidase activity, thyroperoxidase activity Definition: Catalysis of the reaction: iodide + H2O2 = iodine + 2 H2O. Sources: RHEA:23336 Relationships: is a type of GO:0140905